{
  "gene_name": "Astrotactin-2",
  "gene": "UniProtKB:O75129",
  "term_label": "neuron migration",
  "gene_symbol": "ASTN2",
  "term_id": "GO:0001764"
}